{
  "gene_name": "Stalled ribosome sensor GCN1",
  "gene_symbol": "GCN1",
  "term_id": "GO:0005829",
  "gene": "UniProtKB:Q92616",
  "term_label": "cytosol"
}